{
  "gene_symbol": "SMIM36",
  "gene": "UniProtKB:A0A1B0GVT2",
  "term_label": "Unknown biological process",
  "term_id": "UNKNOWN:0002",
  "gene_name": "Small integral membrane protein 36"
}